kinetochore adaptor activity [GO:0140483] (molecular function) Definition: The binding activity of a protein that brings the kinetochore and another molecule into contact, permitting those molecules to function in a coordinated way. Also known as: inner kinetochore adaptor activity, outer kinetochore adaptor activity References: PMID:22521786 Relationships: is a type of GO:0030674